ganglioside binding [GO:0035594] (molecular function) Sources: GOC:yaf Subtypes: ganglioside GM1 binding [GO:1905573], ganglioside GM2 binding [GO:1905574], ganglioside GM3 binding [GO:1905575], ganglioside GT1b binding [GO:1905576], ganglioside GP1c binding [GO:1905577] Definition: Binding to a ganglioside, a ceramide oligosaccharide carrying in addition to other sugar residues, one or more sialic acid residues. Relationships: is a type of GO:0043208; is a type of ceramide binding [GO:0097001]